{
  "gene_symbol": "ELOA2",
  "term_label": "Unknown biological process",
  "gene_name": "Elongin-A2",
  "term_id": "UNKNOWN:0002",
  "gene": "UniProtKB:Q8IYF1"
}